{
  "gene": "UniProtKB:Q96JS3",
  "term_id": "UNKNOWN:0002",
  "gene_symbol": "PGBD1",
  "term_label": "Unknown biological process",
  "gene_name": "PiggyBac transposable element-derived protein 1"
}